regulation of establishment of protein localization to chromosome [GO:0070202] (biological process) Subtypes: regulation of establishment of protein localization to telomere [GO:0070203] Also known as: regulation of establishment of protein localisation to chromosome Sources: GOC:BHF, GOC:mah Definition: Any process that modulates the frequency, rate or extent of the directed movement of a protein to a specific location on a chromosome. Relationships: is a type of regulation of establishment of protein localization [GO:0070201]; regulates establishment of protein localization to chromosome [GO:0070199]